regulation of Golgi calcium ion export [GO:1901472] (biological process) Sources: GOC:TermGenie Relationships: is a type of regulation of release of sequestered calcium ion into cytosol [GO:0051279]; regulates GO:0061454 Definition: Any process that modulates the frequency, rate or extent of Golgi calcium ion export.